{
  "term_id": "GO:0005794",
  "gene": "UniProtKB:Q8N1N2",
  "gene_symbol": "DYNAP",
  "gene_name": "Dynactin-associated protein",
  "term_label": "Golgi apparatus"
}